ADP-heptose-lipopolysaccharide heptosyltransferase activity [GO:0008713] (molecular function) Sources: RHEA:74071 Definition: Catalysis of the reaction: heptosyl-KDO2-lipid A + ADP-L-glycero-beta-D-manno-heptose = heptosyl2-KDO2-lipid A + ADP + H+. Relationships: is a type of lipopolysaccharide heptosyltransferase activity [GO:0008920] Also known as: ADP-heptose:LPS heptosyltransferase activity